glucagon-like peptide 1 receptor activity [GO:0044508] (molecular function) References: PMID:12529935 Sources: GOC:jl Relationships: is a type of G protein-coupled peptide receptor activity [GO:0008528] Definition: Combining with glucagon-like peptide 1 and transmitting the signal across the membrane by activating an associated G-protein.